{
  "term_label": "Unknown biological process",
  "gene_symbol": "TTC13",
  "gene": "UniProtKB:Q8NBP0",
  "term_id": "UNKNOWN:0002",
  "gene_name": "Tetratricopeptide repeat protein 13"
}